homoserine kinase activity [GO:0004413] (MF) Sources: EC:2.7.1.39, RHEA:13985 Also known as: ATP:L-homoserine O-phosphotransferase activity, HSK, homoserine kinase (phosphorylating) Definition: Catalysis of the reaction: L-homoserine + ATP = O-phospho-L-homoserine + ADP + 2 H+. Relationships: is_a phosphotransferase activity, alcohol group as acceptor [GO:0016773]; is a type of amino acid kinase activity [GO:0019202]